regulation of cerebellar neuron development [GO:1905079] (BP) References: PMID:26609159 Sources: GOC:TermGenie, GO_REF:0000058 Definition: Any process that modulates the frequency, rate or extent of cerebellar neuron development. Relationships: is a type of regulation of neuron differentiation [GO:0045664]; is a type of regulation of cell development [GO:0060284]; regulates cerebellar neuron development [GO:0098749] Subtypes: negative regulation of cerebellar neuron development [GO:1905080], positive regulation of cerebellar neuron development [GO:1905081]